{
  "gene_name": "Unconventional myosin-Vb",
  "gene": "UniProtKB:Q9ULV0",
  "term_label": "actin cytoskeleton",
  "gene_symbol": "MYO5B",
  "term_id": "GO:0015629"
}